positive regulation of acrosomal vesicle exocytosis [GO:2000368] (biological process) Definition: Any process that activates or increases the frequency, rate or extent of acrosomal vesicle exocytosis. Sources: GOC:obol Relationships: is_a GO:0045956; is a type of positive regulation of reproductive process [GO:2000243]; is a type of GO:2000367; positively regulates acrosomal vesicle exocytosis [GO:0060478] Also known as: positive regulation of acrosome exocytosis, positive regulation of acrosomal granule exocytosis